{
  "gene": "UniProtKB:P14651",
  "term_label": "DNA-binding transcription factor activity, RNA polymerase II-specific",
  "gene_name": "Homeobox protein Hox-B3",
  "gene_symbol": "HOXB3",
  "term_id": "GO:0000981"
}